{
  "gene_symbol": "KLK7",
  "gene": "UniProtKB:P49862",
  "term_id": "GO:0005615",
  "term_label": "extracellular space",
  "gene_name": "Kallikrein-7"
}